{
  "gene_symbol": "KPNA5",
  "term_label": "NLS-bearing protein import into nucleus",
  "gene": "UniProtKB:O15131",
  "term_id": "GO:0006607",
  "gene_name": "Importin subunit alpha-6"
}